basal cortex [GO:0045180] (cellular component) Sources: GOC:bf Relationships: is a type of cell cortex region [GO:0099738]; is part of GO:0045178 Definition: The region that lies just beneath the plasma membrane on the basal edge of a cell.